{
  "gene_symbol": "BRINP3",
  "term_label": "central nervous system neuron differentiation",
  "gene_name": "BMP_retinoic acid-inducible neural-specific protein 3",
  "gene": "UniProtKB:Q76B58",
  "term_id": "GO:0021953"
}